{
  "term_id": "GO:0030877",
  "gene": "UniProtKB:O15169",
  "term_label": "beta-catenin destruction complex",
  "gene_symbol": "AXIN1",
  "gene_name": "Axin-1"
}